{
  "gene_name": "Rab5 GDP_GTP exchange factor",
  "gene": "UniProtKB:Q9UJ41",
  "term_label": "guanyl-nucleotide exchange factor activity",
  "gene_symbol": "RABGEF1",
  "term_id": "GO:0005085"
}